{
  "gene_symbol": "STX8",
  "term_label": "SNARE binding",
  "term_id": "GO:0000149",
  "gene": "UniProtKB:Q9UNK0",
  "gene_name": "Syntaxin-8"
}